{
  "term_label": "ciliary basal body",
  "gene": "UniProtKB:Q8NHH1",
  "gene_name": "Tubulin polyglutamylase TTLL11",
  "term_id": "GO:0036064",
  "gene_symbol": "TTLL11"
}